achromobactin transport [GO:0042935] (biological process) Relationships: is a type of GO:0015850; is a type of GO:0015891; is a type of GO:0042886; is a type of GO:0046942 Definition: The directed movement of achromobactin, a citrate siderophore, into, out of or within a cell, or between cells, by means of some agent such as a transporter or pore. References: PMID:10928541 Sources: GOC:jl